{
  "term_label": "nucleoplasm",
  "term_id": "GO:0005654",
  "gene_name": "Cytosolic phospholipase A2 gamma",
  "gene": "UniProtKB:Q9UP65",
  "gene_symbol": "PLA2G4C"
}